virus-like capsid [GO:0170047] (cellular component) Definition: A protein coat that surrounds nucleic acid to form a structure similar to a virus capsid. Virus-like capsids are non-infectious and are encoded by endogenous (non-viral) genes. Fly and tetrapod Arc (ancestrally-related to retrotransposon Gag) are examples of proteins that can self-assemble into capsid-like structures which encapsulate Arc mRNA and mediate the intercellular transmission of RNA. References: PMID:29328916 Also known as: virus-like particle Relationships: is_a cellular anatomical structure [GO:0110165]